{
  "term_label": "Unknown biological process",
  "term_id": "UNKNOWN:0002",
  "gene_symbol": "LINC03042",
  "gene": "UniProtKB:Q6ZUL3",
  "gene_name": "Uncharacterized protein LINC03042"
}